{
  "term_label": "plasma membrane",
  "gene_name": "Ankyrin repeat domain-containing protein 13B",
  "gene_symbol": "ANKRD13B",
  "gene": "UniProtKB:Q86YJ7",
  "term_id": "GO:0005886"
}